trichome differentiation [GO:0010026] (biological process) Subtypes: seed trichome differentiation [GO:0090376] Definition: The process in which a relatively unspecialized epidermal cell acquires the specialized features of a trichome cell. An example of this process is found in Arabidopsis thaliana. Also known as: trichome cell differentiation Relationships: is a type of cell differentiation [GO:0030154]; is part of plant epidermis development [GO:0090558] References: PMID:9367433 Sources: GOC:mtg_sensu